ERBB4-EGFR complex [GO:0038139] (cellular component) Definition: A heterodimeric complex between the tyrosine kinase receptors ERBB4 (also called HER4) and epidermal growth factor receptor (EGFR/ERBB1). References: PMID:16460914 Sources: GOC:signaling Also known as: EGFR-ERBB4 complex, ERBB4:EGFR heterodimer Relationships: is a type of plasma membrane signaling receptor complex [GO:0098802]